monoatomic anion channel activity [GO:0005253] (molecular function) Definition: Enables the energy-independent facilitated diffusion of a monoatomic anion through a transmembrane aqueous pore or channel. Regulation: negatively regulated by negative regulation of anion channel activity [GO:0010360]; positively regulated by positive regulation of anion channel activity [GO:1901529] Relationships: is a type of monoatomic ion channel activity [GO:0005216]; is a type of monoatomic anion transmembrane transporter activity [GO:0008509] Also known as: anion channel activity, non-selective anion channel activity Sources: GOC:dph, GOC:mtg_transport, GOC:pr, ISBN:0815340729 Subtypes: volume-sensitive anion channel activity [GO:0005225], chloride channel activity [GO:0005254], voltage-gated monoatomic anion channel activity [GO:0008308], fluoride channel activity [GO:0062054], GO:0099095, iodide channel activity [GO:0160081]